{
  "gene": "UniProtKB:Q5JWR5",
  "term_label": "endosome",
  "gene_symbol": "DOP1A",
  "gene_name": "Protein dopey-1",
  "term_id": "GO:0005768"
}